S-nitrosoglutathione binding [GO:0035730] (molecular function) Definition: Binding to S-nitrosoglutathione, a nitrosothiol considered to be a natural nitric oxide (NO) donor involved in S-nitrosylation, and in the storage and transport of nitric oxide in biological systems. Sources: GOC:BHF Also known as: GSNO binding Relationships: is a type of anion binding [GO:0043168]; is a type of sulfur compound binding [GO:1901681]